{
  "term_label": "cell adhesion",
  "gene_symbol": "PCDHGC5",
  "gene_name": "Protocadherin gamma-C5",
  "term_id": "GO:0007155",
  "gene": "UniProtKB:Q9Y5F6"
}